cell differentiation in hindbrain [GO:0021533] (biological process) Definition: The process in which relatively unspecialized cells acquire specialized structural and/or functional features that characterize the mature cells of the hindbrain. Differentiation includes the processes involved in commitment of a cell to a specific fate. Subtypes: GO:0021701, cerebellar Purkinje cell differentiation [GO:0021702], GO:0021707, GO:0021708, cerebellar basket cell differentiation [GO:0021709], cerebellar stellate cell differentiation [GO:0021710], cerebellar unipolar brush cell differentiation [GO:0021711], candelabrum cell differentiation [GO:0021712], GO:0021755 Relationships: is a type of cell differentiation [GO:0030154]; is part of GO:0030902 Sources: GOC:cls, GOC:dgh, GOC:dph, GOC:jid, GO_REF:0000021